{
  "gene_symbol": "GPATCH11",
  "term_label": "Unknown biological process",
  "gene_name": "G patch domain-containing protein 11",
  "gene": "UniProtKB:Q8N954",
  "term_id": "UNKNOWN:0002"
}